{
  "term_label": "Unknown biological process",
  "gene_name": "BTB_POZ domain-containing protein 19",
  "gene_symbol": "BTBD19",
  "term_id": "UNKNOWN:0002",
  "gene": "UniProtKB:C9JJ37"
}